maintenance of location [GO:0051235] (BP) Definition: Any process in which a cell, substance or cellular entity, such as a protein complex or organelle, is maintained in a location and prevented from moving elsewhere. Sources: GOC:ai, GOC:dph, GOC:tb Also known as: maintenance of localization, retention, sequestering, storage Relationships: is a type of GO:0051179 Subtypes: GO:0045185, GO:0051237, maintenance of location in cell [GO:0051651], maintenance of protein complex location [GO:0098544]